{
  "term_id": "GO:0045214",
  "gene_symbol": "CSRP3",
  "gene": "UniProtKB:P50461",
  "gene_name": "Cysteine and glycine-rich protein 3",
  "term_label": "sarcomere organization"
}